{
  "gene_symbol": "KDM4E",
  "term_label": "regulation of gene expression",
  "gene_name": "Lysine-specific demethylase 4E",
  "gene": "UniProtKB:B2RXH2",
  "term_id": "GO:0010468"
}